cysteinyl-tRNA aminoacylation [GO:0006423] (biological process) Sources: GOC:mcc, ISBN:0716730510 Relationships: is a type of tRNA aminoacylation for protein translation [GO:0006418] Definition: The process of coupling cysteine to cysteinyl-tRNA, catalyzed by cysteinyl-tRNA synthetase. A cysteinyl-tRNA synthetase is a class-I synthetase. The activated amino acid is transferred to the 2'-OH group of a cysteine-accetping tRNA. The 2'-O-aminoacyl-tRNA will ultimately migrate to the 3' position via transesterification. Subtypes: mitochondrial cysteinyl-tRNA aminoacylation [GO:0070147]